{
  "term_label": "precatalytic spliceosome",
  "gene_symbol": "RBMX2",
  "gene_name": "RNA-binding motif protein, X-linked 2",
  "gene": "UniProtKB:Q9Y388",
  "term_id": "GO:0071011"
}